G protein-coupled neurotransmitter receptor activity [GO:0099528] (molecular function) Also known as: G-protein coupled neurotransmitter receptor activity Subtypes: GO:0016907, G protein-coupled neurotransmitter receptor activity involved in regulation of postsynaptic cytosolic calcium ion concentration [GO:0098872], G protein-coupled neurotransmitter receptor activity involved in regulation of postsynaptic membrane potential [GO:0099579], G protein-coupled neurotransmitter receptor activity involved in regulation of presynaptic membrane potential [GO:0150047], G protein-coupled glycine receptor activity [GO:0160079] Relationships: is a type of G protein-coupled receptor activity [GO:0004930]; is a type of GO:0030594 Definition: Combining with a neurotransmitter and transmitting the signal across the membrane by activating an associated G-protein; promotes the exchange of GDP for GTP on the alpha subunit of a heterotrimeric G-protein complex. Sources: GOC:bf, GOC:fj, GOC:mah